maintenance of protein location [GO:0045185] (BP) Subtypes: maintenance of protein location in cell [GO:0032507], maintenance of protein location in extracellular region [GO:0071694] Also known as: active protein retrieval, protein retention, protein sequestering, maintenance of protein localization Relationships: is a type of maintenance of location [GO:0051235]; is part of intracellular protein localization [GO:0008104] Sources: GOC:bf Definition: Any process in which a protein is maintained in a location and prevented from moving elsewhere. These include sequestration, stabilization to prevent transport elsewhere and the active retrieval of proteins that do move away.